chlorophyll a biosynthetic process via phytyl diphosphate [GO:0033311] (biological process) Definition: The chemical reactions and pathways leading to the formation of chlorophyll a, via the intermediate phytyl diphosphate. Sources: GOC:mah, MetaCyc:PWY-5086 Also known as: chlorophyll a anabolism via phytyl diphosphate, chlorophyll a biosynthesis via phytyl diphosphate, chlorophyll a biosynthetic process via phytyl-PP, chlorophyll a formation via phytyl chlorophyll a formation via phytyl-PP, chlorophyll a synthesis via phytyl diphosphate Relationships: is a type of chlorophyll a biosynthetic process [GO:0033305]